DNA polymerase III, core complex [GO:0044776] (CC) Definition: The DNA polymerase III core complex consists of the alpha,epsilon and theta subunits and is carries out the polymerase and the 3'-5' exonuclease proofreading activities. Sources: GOC:jl, UniProt:P06710 Relationships: is a type of GO:0140513; is part of GO:0009360